{
  "term_id": "GO:0003714",
  "gene": "UniProtKB:P25685",
  "gene_symbol": "DNAJB1",
  "term_label": "transcription corepressor activity",
  "gene_name": "DnaJ homolog subfamily B member 1"
}